{
  "gene_name": "Cytoskeleton-associated protein 2-like",
  "term_label": "mitotic spindle",
  "gene_symbol": "CKAP2L",
  "gene": "UniProtKB:Q8IYA6",
  "term_id": "GO:0072686"
}